{
  "term_id": "GO:0005783",
  "gene_symbol": "DDRGK1",
  "term_label": "endoplasmic reticulum",
  "gene_name": "DDRGK domain-containing protein 1",
  "gene": "UniProtKB:Q96HY6"
}